{
  "gene_symbol": "ZNF14",
  "term_label": "regulation of transcription by RNA polymerase II",
  "gene": "UniProtKB:P17017",
  "term_id": "GO:0006357",
  "gene_name": "Zinc finger protein 14"
}